{
  "term_id": "GO:0000398",
  "term_label": "mRNA splicing, via spliceosome",
  "gene_name": "U11_U12 small nuclear ribonucleoprotein 35 kDa protein",
  "gene_symbol": "SNRNP35",
  "gene": "UniProtKB:Q16560"
}